{
  "gene_symbol": "POLR2G",
  "term_label": "translation initiation factor binding",
  "gene_name": "DNA-directed RNA polymerase II subunit RPB7",
  "gene": "UniProtKB:P62487",
  "term_id": "GO:0031369"
}